cellularization cleavage furrow [GO:0110070] (cellular component) Definition: A plasma membrane invagination at the site of separation of a multi-nucleate cell or syncytium into individual cells. Relationships: is a type of plasma membrane region [GO:0098590] References: PMID:27226317 Sources: GOC:ha